{
  "gene_name": "Carboxypeptidase Q",
  "term_label": "extracellular space",
  "term_id": "GO:0005615",
  "gene_symbol": "CPQ",
  "gene": "UniProtKB:Q9Y646"
}